{
  "gene": "UniProtKB:P0DMW5",
  "gene_symbol": "SMIM10L2B",
  "term_label": "Unknown molecular function",
  "gene_name": "Small integral membrane protein 10-like protein 2B",
  "term_id": "UNKNOWN:0001"
}